{
  "gene_symbol": "PAGR1",
  "gene": "UniProtKB:Q9BTK6",
  "gene_name": "PAXIP1-associated glutamate-rich protein 1",
  "term_id": "GO:0033148",
  "term_label": "positive regulation of intracellular estrogen receptor signaling pathway"
}